{
  "gene": "UniProtKB:Q9Y548",
  "term_id": "UNKNOWN:0001",
  "term_label": "Unknown molecular function",
  "gene_symbol": "YIPF1",
  "gene_name": "Protein YIPF1"
}